filopodium [GO:0030175] (cellular component) Definition: Thin, stiff, actin-based protrusion extended by the leading edge of a motile cell such as a crawling fibroblast or amoeba, or an axonal or dendritic growth cone, or a dendritic shaft. Sources: GOC:mah, GOC:pr, ISBN:0815316194 Note: A filopodium may be approximately 0.1 um wide, 5-10 um long, and up to 50 um long in axon growth cones; contain a loose bundle of about 20 actin filaments oriented with their plus ends pointing outward. Note that filopodia on dendritic shafts are distinct from other types of filopodia (even those found in dendritic growth cones) and may react differently to stimuli, as shown in PMID:12904473. Relationships: is a type of GO:0098858 Subtypes: GO:1902737, growth cone filopodium [GO:1990812]